{
  "term_id": "GO:0000146",
  "gene": "UniProtKB:Q9Y4I1",
  "gene_name": "Unconventional myosin-Va",
  "term_label": "microfilament motor activity",
  "gene_symbol": "MYO5A"
}